{
  "gene_name": "Tudor and KH domain-containing protein",
  "gene": "UniProtKB:Q9Y2W6",
  "term_id": "GO:0030719",
  "gene_symbol": "TDRKH",
  "term_label": "P granule organization"
}